vagus nerve morphogenesis [GO:0021644] (biological process) Relationships: is a type of cranial nerve morphogenesis [GO:0021602]; is part of vagus nerve development [GO:0021564] Also known as: CN X morphogenesis Sources: GOC:cls, GOC:dgh, GOC:dph, GOC:jid, GO_REF:0000021 Definition: The process in which the anatomical structure of the vagus nerve is generated and organized. This nerve is primarily sensory but also has visceromotor components. It originates in the brain stem and controls many autonomic functions of the heart, lungs, stomach, pharynx, larynx, trachea, esophagus and other gastrointestinal tract components. It controls some motor functions such as speech. The sensory branches mediate sensation from the pharynx, larynx, thorax and abdomen; it also innervates taste buds in the epiglottis.